{
  "gene_symbol": "PCDHA2",
  "gene_name": "Protocadherin alpha-2",
  "term_id": "GO:0050839",
  "gene": "UniProtKB:Q9Y5H9",
  "term_label": "cell adhesion molecule binding"
}